{
  "term_label": "positive regulation of receptor signaling pathway via JAK-STAT",
  "gene": "UniProtKB:P01242",
  "term_id": "GO:0046427",
  "gene_symbol": "GH2",
  "gene_name": "Growth hormone variant"
}